regulation of protein secretion [GO:0050708] (biological process) Definition: Any process that modulates the frequency, rate or extent of the controlled release of a protein from a cell. Sources: GOC:ai Relationships: is_a GO:0051223; is a type of regulation of secretion by cell [GO:1903530]; regulates protein secretion [GO:0009306] Subtypes: negative regulation of protein secretion [GO:0050709], positive regulation of protein secretion [GO:0050714], regulation of insulin secretion [GO:0050796], regulation of Wnt protein secretion [GO:0061356], regulation of adiponectin secretion [GO:0070163], GO:0090182, regulation of renin secretion into blood stream [GO:1900133], regulation of pancreatic amylase secretion [GO:1902276], regulation of pancreatic trypsinogen secretion [GO:1904242], regulation of matrix metallopeptidase secretion [GO:1904464], regulation of BMP secretion [GO:2001284]